{
  "gene_symbol": "A0A0G2JPN4",
  "gene": "UniProtKB:A0A0G2JPN4",
  "term_label": "Unknown cellular component",
  "gene_name": "Uncharacterized protein",
  "term_id": "UNKNOWN:0003"
}